{
  "term_id": "GO:0043495",
  "gene_name": "Putative PDZ domain-containing protein PDZK1P1",
  "gene": "UniProtKB:A8MUH7",
  "term_label": "protein-membrane adaptor activity",
  "gene_symbol": "PDZK1P1"
}